{
  "gene_name": "Centrosomal protein of 164 kDa",
  "gene": "UniProtKB:Q9UPV0",
  "gene_symbol": "CEP164",
  "term_label": "centrosome",
  "term_id": "GO:0005813"
}